host cell nuclear lamina [GO:0044203] (cellular component) Definition: The fibrous, electron-dense layer lying on the nucleoplasmic side of the inner membrane of a host cell nucleus, composed of lamin filaments. Sources: GOC:jl Relationships: is a type of host cell nuclear part [GO:0044094]; BFO_0000050 host cell nuclear inner membrane [GO:0044201]